{
  "term_label": "TRAMP-dependent tRNA surveillance pathway",
  "gene_symbol": "EXOSC7",
  "gene": "UniProtKB:Q15024",
  "term_id": "GO:0071038",
  "gene_name": "Exosome complex component RRP42"
}